{
  "gene_name": "START domain-containing protein 10",
  "gene_symbol": "STARD10",
  "term_id": "GO:0005829",
  "term_label": "cytosol",
  "gene": "UniProtKB:Q9Y365"
}